autophagosome lumen [GO:0034423] (cellular component) Sources: GOC:autophagy, GOC:rph Relationships: is a type of GO:0005775; is part of autophagosome [GO:0005776] Definition: The volume enclosed within the autophagosome double-membrane. Note: Note that this term should be used for annotating gene products with caution: it should be used only to annotate gene products demonstrated to reside and function normally in the autophagic vacuole lumen, not for molecules that are temporarily found in the lumen prior to degradation. Also known as: autophagic vacuole lumen